RNA polymerase II CTD heptapeptide repeat phosphatase activity [GO:0008420] (molecular function) Relationships: is a type of GO:0004722; is a type of RNA polymerase II CTD heptapeptide repeat modifying activity [GO:0140994] References: PMID:22622228 Subtypes: RNA polymerase II CTD heptapeptide repeat Y1 phosphatase activity [GO:0180004], RNA polymerase II CTD heptapeptide repeat T4 phosphatase activity [GO:0180005], RNA polymerase II CTD heptapeptide repeat S2 phosphatase activity [GO:0180006], RNA polymerase II CTD heptapeptide repeat S5 phosphatase activity [GO:0180007], RNA polymerase II CTD heptapeptide repeat S7 phosphatase activity [GO:0180008] Definition: Catalysis of the reaction: RNA polymerase II large subunit CTD heptapeptide repeat--phospho-L-serine/threonine (consensus YSPTSPS) + H2O = RNA polymerase II large subunit + phosphate. Also known as: CTD phosphatase activity, RNA polymerase II carboxy-terminal domain phosphatase activity